candicidin biosynthetic process [GO:1901127] (biological process) Relationships: is a type of GO:0009058 Sources: GOC:TermGenie, GOC:yaf, UniPathway:UPA00101 Also known as: candicidin anabolism, candicidin biosynthesis, candicidin formation, candicidin synthesis Definition: The chemical reactions and pathways resulting in the formation of candicidin.